flavonoid phytoalexin catabolic process [GO:0046286] (biological process) Definition: The chemical reactions and pathways resulting in the breakdown of flavonoid phytoalexins, a group of water-soluble phenolic derivatives containing a flavan skeleton, which possess antibiotic activity and are produced by plant tissues in response to infection. Also known as: flavonoid phytoalexin breakdown, flavonoid phytoalexin catabolism, flavonoid phytoalexin degradation Sources: GOC:ai Relationships: is a type of GO:0046275; is a type of GO:0052316